inositol pyrophosphate sensor activity [GO:0180043] (molecular function) Definition: Binding to and responding, e.g. by conformational change, to changes in the cellular level of an inositol pyrophosphate. References: PMID:37949217 Relationships: is a type of molecular sensor activity [GO:0140299]